{
  "gene_name": "Homeobox protein Hox-D11",
  "term_id": "GO:0000978",
  "gene_symbol": "HOXD11",
  "gene": "UniProtKB:P31277",
  "term_label": "RNA polymerase II cis-regulatory region sequence-specific DNA binding"
}